protein localization to nuclear envelope [GO:0090435] (biological process) Sources: GOC:tb Definition: A process in which a protein is transported to, or maintained at, a location within a nuclear envelope. Also known as: protein localization in nuclear envelope Relationships: is a type of protein localization to nucleus [GO:0034504] Subtypes: protein localization to nuclear inner membrane [GO:0036228], GO:0090204